{
  "gene": "UniProtKB:Q15047",
  "term_id": "GO:0005634",
  "gene_name": "Histone-lysine N-methyltransferase SETDB1",
  "term_label": "nucleus",
  "gene_symbol": "SETDB1"
}